CDP-glucose 4,6-dehydratase activity [GO:0047733] (molecular function) Also known as: CDP-glucose 4,6-hydro-lyase (CDP-4-dehydro-6-deoxy-D-glucose-forming), CDP-glucose 4,6-hydro-lyase activity, CDPglucose 4,6-dehydratase activity, CDPglucose 4,6-hydro-lyase activity, cytidine diphosphoglucose oxidoreductase activity Definition: Catalysis of the reaction: CDP-D-glucose = CDP-4-dehydro-6-deoxy-D-glucose + H2O. Sources: EC:4.2.1.45, RHEA:17153 Relationships: is a type of hydro-lyase activity [GO:0016836]